anaerobic amino acid catabolic process [GO:0019665] (biological process) Definition: The anaerobic chemical reactions and pathways resulting in the breakdown of amino acids, yielding energy in the form of ATP. Sources: GOC:curators, GOC:jl Also known as: amino acid fermentation Relationships: is a type of GO:0006113; is a type of amino acid catabolic process [GO:0009063] Subtypes: L-lysine fermentation [GO:0019475], anaerobic L-alanine catabolic process [GO:0019667], GO:0019668, GO:0019669, anaerobic L-glutamate catabolic process [GO:0019670]